{
  "term_id": "GO:0071261",
  "gene": "UniProtKB:P60059",
  "gene_symbol": "SEC61G",
  "term_label": "Ssh1 translocon complex",
  "gene_name": "Protein transport protein Sec61 subunit gamma"
}